negative regulation of intracellular lipid transport [GO:0032378] (BP) Subtypes: negative regulation of intracellular sterol transport [GO:0032381] Sources: GOC:mah Relationships: is_a negative regulation of lipid transport [GO:0032369]; is a type of GO:0032377; is a type of negative regulation of intracellular transport [GO:0032387]; RO_0002212 intracellular lipid transport [GO:0032365] Definition: Any process that stops, prevents, or reduces the frequency, rate or extent of the directed movement of lipids within cells. Also known as: down regulation of intracellular lipid transport, down-regulation of intracellular lipid transport, downregulation of intracellular lipid transport, inhibition of intracellular lipid transport